{
  "term_label": "minus-end-directed microtubule motor activity",
  "gene_name": "Dynein axonemal heavy chain 17",
  "gene_symbol": "DNAH17",
  "term_id": "GO:0008569",
  "gene": "UniProtKB:Q9UFH2"
}